{
  "gene_name": "Nuclear receptor subfamily 1 group I member 2",
  "gene": "UniProtKB:O75469",
  "term_label": "cell differentiation",
  "term_id": "GO:0030154",
  "gene_symbol": "NR1I2"
}